response to G2 transition size control checkpoint signaling [GO:0072452] (biological process) Sources: GOC:mtg_cell_cycle Relationships: is a type of response to cell size control checkpoint signaling [GO:0072470] Also known as: G2/M transition size control checkpoint effector process, response to G2/M transition size control checkpoint signaling, response to mitotic cell cycle G2/M transition size control checkpoint signaling, response to signal involved in G2/M transition size control checkpoint Definition: A process that occurs in response to signals generated as a result of G2/M transition size control checkpoint signaling.